positive regulation of aeciospore formation [GO:0075249] (biological process) Relationships: is a type of GO:0043945; is a type of regulation of aeciospore formation [GO:0075248]; RO_0002213 GO:0075247 Sources: GOC:pamgo_curators Definition: Any process that activates, maintains or increases the frequency, rate or extent of aeciospore formation, a process in which a dikaryotic spore of typically a rust fungus is produced in an aecium.